{
  "gene_name": "rRNA N6-adenosine-methyltransferase ZCCHC4",
  "gene_symbol": "ZCCHC4",
  "term_label": "cytoplasm",
  "term_id": "GO:0005737",
  "gene": "UniProtKB:Q9H5U6"
}